{
  "gene_name": "Regulator of microtubule dynamics protein 3",
  "term_id": "GO:0005739",
  "gene": "UniProtKB:Q96TC7",
  "gene_symbol": "RMDN3",
  "term_label": "mitochondrion"
}